{
  "gene_symbol": "FBXL21P",
  "term_label": "SCF-dependent proteasomal ubiquitin-dependent protein catabolic process",
  "gene_name": "Putative F-box_LRR-repeat protein 21",
  "term_id": "GO:0031146",
  "gene": "UniProtKB:Q9UKT6"
}